amyloid-beta complex [GO:0106003] (cellular component) References: PMID:18568035 Sources: GOC:bhm Definition: Protein complex involved in modulation of signaling and synaptic function in the brain, predominantly in the cerebral cortex and hippocampus. Forms dimers and multimers of amyloid beta peptide 40 and peptide 42 (proteolytic cleavage products of amyloid beta A4 protein, also known as amyloid beta precursor protein). Mostly found in the extracellular space with a proportion occurring as membrane-bound species. Influences synaptic plasticity through various receptors, mediates dendritic spine loss leading to decreased synapse density, inhibits long-term potentiation (LTP) and enhances long-term depression (LTD). Soluble multimeric form is the main pathogenic species linked to Alzheimer's disease. Also known as: Abeta complex, amyloid beta complex, beta amyloid complex, beta-amyloid complex, betaA complex, ADDL complex, Abeta-derived diffusible ligand complex, amyloid beta dimer, amyloid beta heterodimer, amyloid beta heterooligomer, amyloid beta heterotrimer, amyloid beta homodimer, amyloid beta homooligomer, amyloid beta homotrimer, amyloid beta oligomer, amyloid beta trimer, amyloid-beta protein 40 complex, amyloid-beta protein 40/42 complex, amyloid-beta protein 42 complex, heterodimer of amyloid beta protein, heterooligomer of amyloid beta protein, heterotrimer of amyloid beta protein, homodimer of amyloid beta protein, homooligomer of amyloid beta protein, homotrimer of amyloid beta protein Relationships: is a type of protein-containing complex [GO:0032991] Note: An example is Protein 40 of APP (P05067-PRO_0000000093) in PMID:18568035 (inferred by direct assay).